{
  "term_id": "GO:0004674",
  "gene": "UniProtKB:Q13627",
  "gene_name": "Dual specificity tyrosine-phosphorylation-regulated kinase 1A",
  "gene_symbol": "DYRK1A",
  "term_label": "protein serine/threonine kinase activity"
}